{
  "gene": "UniProtKB:O15391",
  "gene_name": "Transcription factor YY2",
  "term_label": "chromatin",
  "term_id": "GO:0000785",
  "gene_symbol": "YY2"
}